{
  "term_id": "GO:0033234",
  "gene_name": "Fibrous sheath CABYR-binding protein",
  "gene": "UniProtKB:Q5H9T9",
  "gene_symbol": "FSCB",
  "term_label": "negative regulation of protein sumoylation"
}